{
  "term_id": "GO:0010845",
  "gene": "UniProtKB:Q9NQV7",
  "gene_name": "Histone-lysine N-methyltransferase PRDM9",
  "term_label": "positive regulation of reciprocal meiotic recombination",
  "gene_symbol": "PRDM9"
}